regulation of meiosis I spindle assembly checkpoint [GO:1905325] (biological process) Relationships: is_a regulation of meiosis I [GO:0060631]; is a type of regulation of spindle checkpoint [GO:0090231]; is a type of GO:1902102; RO_0002211 meiosis I spindle assembly checkpoint signaling [GO:1905318] Subtypes: positive regulation of meiosis I spindle assembly checkpoint [GO:1905326] References: PMID:26483559 Sources: GOC:TermGenie, GO_REF:0000058 Definition: Any process that modulates the frequency, rate or extent of the meiosis I spindle assembly checkpoint.